{
  "gene_symbol": "GK2",
  "gene": "UniProtKB:Q14410",
  "term_label": "triglyceride metabolic process",
  "gene_name": "Glycerol kinase 2",
  "term_id": "GO:0006641"
}